transferase activity, transferring one-carbon groups [GO:0016741] (molecular function) Definition: Catalysis of the transfer of a one-carbon group from one compound (donor) to another (acceptor). Sources: GOC:jl, ISBN:0198506732 Also known as: methyltransferase activity Relationships: is_a transferase activity [GO:0016740] Subtypes: methyltransferase activity [GO:0008168], amidinotransferase activity [GO:0015067], hydroxymethyl-, formyl- and related transferase activity [GO:0016742], carboxyl- or carbamoyltransferase activity [GO:0016743]